wing and notum subfield formation [GO:0035309] (biological process) References: PMID:10860999 Relationships: is a type of regionalization [GO:0003002]; is part of wing disc development [GO:0035220] Definition: The regionalization process that subdivides the wing imaginal disc into the wing and notum (body wall) subfields, thus determining whether cells ultimately differentiate wing or notum-specific structures.